cytoplasmic side of endoplasmic reticulum membrane [GO:0098554] (cellular component) Relationships: is a type of cytoplasmic side of membrane [GO:0098562]; is part of endoplasmic reticulum membrane [GO:0005789] Definition: The side (leaflet) of the plasma membrane that faces the cytoplasm. Sources: GOC:ab, GOC:dos Subtypes: cytoplasmic side of rough endoplasmic reticulum membrane [GO:0098556], cytoplasmic side of smooth endoplasmic reticulum membrane [GO:0098557]